{
  "gene_name": "Pre-mRNA-splicing factor RBM22",
  "gene": "UniProtKB:Q9NW64",
  "gene_symbol": "RBM22",
  "term_label": "U6 snRNA binding",
  "term_id": "GO:0017070"
}